{
  "gene": "UniProtKB:Q8NGP8",
  "term_label": "odorant binding",
  "gene_name": "Olfactory receptor 5M1",
  "term_id": "GO:0005549",
  "gene_symbol": "OR5M1"
}